{
  "gene_symbol": "EMX2",
  "gene": "UniProtKB:Q04743",
  "gene_name": "Homeobox protein EMX2",
  "term_id": "GO:0030182",
  "term_label": "neuron differentiation"
}